L-malate dehydrogenase (NADP+) activity [GO:0046554] (molecular function) Definition: Catalysis of the reaction: (S)-malate + NADP+ = oxaloacetate + NADPH + H+. Sources: RHEA:10824 Also known as: (S)-malate:NADP+ oxidoreductase activity, NADP malate dehydrogenase activity, NADP-linked malate dehydrogenase activity, NADP-malate dehydrogenase activity, malate NADP dehydrogenase activity, malic dehydrogenase (nicotinamide adenine dinucleotide phosphate) Relationships: is a type of GO:0016615; is a type of oxidoreductase activity, acting on the CH-OH group of donors, NAD or NADP as acceptor [GO:0016616]